{
  "gene_symbol": "GNPNAT1",
  "gene": "UniProtKB:Q96EK6",
  "term_id": "UNKNOWN:0003",
  "gene_name": "Glucosamine 6-phosphate N-acetyltransferase",
  "term_label": "Unknown cellular component"
}